{
  "term_label": "Set1C/COMPASS complex",
  "gene": "UniProtKB:Q15291",
  "term_id": "GO:0048188",
  "gene_symbol": "RBBP5",
  "gene_name": "Retinoblastoma-binding protein 5"
}